{
  "term_label": "cardiac left ventricle formation",
  "gene_symbol": "TBX5",
  "term_id": "GO:0003218",
  "gene_name": "T-box transcription factor TBX5",
  "gene": "UniProtKB:Q99593"
}